{
  "term_label": "intracellular receptor signaling pathway",
  "gene": "UniProtKB:P55055",
  "gene_symbol": "NR1H2",
  "gene_name": "Oxysterols receptor LXR-beta",
  "term_id": "GO:0030522"
}